positive regulation of trypanothione biosynthetic process [GO:1905724] (biological process) Definition: Any process that activates or increases the frequency, rate or extent of trypanothione biosynthetic process. References: PMID:18949025 Sources: GOC:TermGenie, GO_REF:0000058 Also known as: positive regulation of trypanothione anabolism, positive regulation of trypanothione biosynthesis, positive regulation of trypanothione formation, positive regulation of trypanothione synthesis, up regulation of trypanothione anabolism, up regulation of trypanothione biosynthesis, up regulation of trypanothione biosynthetic process, up regulation of trypanothione formation, up regulation of trypanothione synthesis, up-regulation of trypanothione anabolism, up-regulation of trypanothione biosynthesis, up-regulation of trypanothione biosynthetic process, up-regulation of trypanothione formation, up-regulation of trypanothione synthesis, upregulation of trypanothione anabolism, upregulation of trypanothione biosynthesis, upregulation of trypanothione biosynthetic process, upregulation of trypanothione formation, upregulation of trypanothione synthesis, activation of trypanothione anabolism, activation of trypanothione biosynthesis, activation of trypanothione biosynthetic process, activation of trypanothione formation, activation of trypanothione synthesis Relationships: is a type of positive regulation of biosynthetic process [GO:0009891]; is_a regulation of trypanothione biosynthetic process [GO:1905722]; positively regulates GO:0019342